{
  "gene_name": "Prosaposin receptor GPR37",
  "term_id": "GO:0043410",
  "term_label": "positive regulation of MAPK cascade",
  "gene_symbol": "GPR37",
  "gene": "UniProtKB:O15354"
}